{
  "gene_symbol": "IGHV2-70",
  "term_label": "antigen binding",
  "gene_name": "Immunoglobulin heavy variable 2-70",
  "term_id": "GO:0003823",
  "gene": "UniProtKB:P01814"
}